{
  "gene": "UniProtKB:Q14641",
  "gene_name": "Early placenta insulin-like peptide",
  "term_id": "UNKNOWN:0001",
  "gene_symbol": "INSL4",
  "term_label": "Unknown molecular function"
}